{
  "gene": "UniProtKB:Q68D10",
  "gene_name": "Protein SPT2 homolog",
  "term_label": "nucleosome assembly",
  "term_id": "GO:0006334",
  "gene_symbol": "SPTY2D1"
}